{
  "gene_symbol": "LYPD2",
  "gene_name": "Ly6_PLAUR domain-containing protein 2",
  "term_id": "UNKNOWN:0001",
  "gene": "UniProtKB:Q6UXB3",
  "term_label": "Unknown molecular function"
}